{
  "term_id": "GO:0035567",
  "gene_symbol": "FZD10",
  "gene": "UniProtKB:Q9ULW2",
  "term_label": "non-canonical Wnt signaling pathway",
  "gene_name": "Frizzled-10"
}